fucose:proton symporter activity [GO:0015535] (molecular function) Definition: Enables the transfer of a solute or solutes from one side of a membrane to the other according to the reaction: fucose(out) + H+(out) = fucose(in) + H+(in). Sources: TC:2.A.1.7.1 Also known as: fucose:hydrogen symporter activity Relationships: is a type of GO:0009679; is a type of fucose transmembrane transporter activity [GO:0015150]